{
  "gene_name": "Interleukin-20",
  "term_id": "GO:0005615",
  "gene_symbol": "IL20",
  "gene": "UniProtKB:Q9NYY1",
  "term_label": "extracellular space"
}